{
  "term_label": "Unknown molecular function",
  "gene_name": "Protein FAM199X",
  "gene_symbol": "FAM199X",
  "gene": "UniProtKB:Q6PEV8",
  "term_id": "UNKNOWN:0001"
}